endothelial microparticle [GO:0072563] (cellular component) Relationships: is a type of blood microparticle [GO:0072562] Definition: A blood microparticle that is derived from, and contains membrane receptors as well as other proteins characteristic of, an endothelial cell. References: PMID:16373184 Sources: GOC:BHF, GOC:mah